cell morphogenesis involved in conjugation with cellular fusion [GO:0000753] (biological process) Relationships: is a type of cell morphogenesis [GO:0000902]; is part of GO:0000747 Also known as: shmoo orientation, shmooing Sources: GOC:clt Definition: The change in form (cell shape and size) that occurs during sexual reproduction in order to facilitate direct contact between the compatible mating types in organisms that undergo conjugation cellular fusion. Regulation: regulated by regulation of cell morphogenesis involved in conjugation with cellular fusion [GO:1905708]